regulation of dorsal/ventral axon guidance [GO:1905815] (biological process) Definition: Any process that modulates the frequency, rate or extent of dorsal/ventral axon guidance. References: PMID:18434533 Sources: GOC:TermGenie, GO_REF:0000058 Subtypes: GO:1905816, positive regulation of dorsal/ventral axon guidance [GO:1905817] Also known as: regulation of dorsal-ventral axon guidance, regulation of dorsal/ventral axon pathfinding, regulation of dorsoventral axon guidance Relationships: is a type of GO:1902667; regulates dorsal/ventral axon guidance [GO:0033563]